{
  "gene": "UniProtKB:Q5W064",
  "gene_symbol": "LIPJ",
  "term_label": "lipase activity",
  "term_id": "GO:0016298",
  "gene_name": "Lipase member J"
}